{
  "term_id": "GO:0000139",
  "gene_name": "Protein O-linked-mannose beta-1,2-N-acetylglucosaminyltransferase 1",
  "term_label": "Golgi membrane",
  "gene_symbol": "POMGNT1",
  "gene": "UniProtKB:Q8WZA1"
}